{
  "term_id": "UNKNOWN:0001",
  "gene": "UniProtKB:Q6PRD7",
  "term_label": "Unknown molecular function",
  "gene_name": "Cementoblastoma-derived protein 1",
  "gene_symbol": "CEMP1"
}